{
  "gene_name": "Zinc finger homeobox protein 2",
  "term_label": "nucleus",
  "term_id": "GO:0005634",
  "gene_symbol": "ZFHX2",
  "gene": "UniProtKB:Q9C0A1"
}